{
  "gene": "UniProtKB:Q8NFJ9",
  "gene_symbol": "BBS1",
  "term_id": "GO:0005113",
  "gene_name": "Bardet-Biedl syndrome 1 protein",
  "term_label": "patched binding"
}